{
  "gene_symbol": "MS4A14",
  "term_id": "GO:0007166",
  "gene": "UniProtKB:Q96JA4",
  "gene_name": "Membrane-spanning 4-domains subfamily A member 14",
  "term_label": "cell surface receptor signaling pathway"
}